nor-spermidine catabolic process [GO:0046205] (BP) Definition: The chemical reactions and pathways resulting in the breakdown of nor-spermidine, a compound related to spermidine, N-(3-aminopropyl)-1,4-diaminobutane. Sources: GOC:ai Also known as: nor-spermidine breakdown, nor-spermidine catabolism, nor-spermidine degradation Relationships: is a type of polyamine catabolic process [GO:0006598]; is a type of GO:0046204